{
  "term_id": "GO:0005615",
  "gene_name": "Lutropin subunit beta",
  "gene_symbol": "LHB",
  "term_label": "extracellular space",
  "gene": "UniProtKB:P01229"
}